{
  "term_id": "GO:0044613",
  "term_label": "nuclear pore central transport channel",
  "gene": "UniProtKB:Q7Z3B4",
  "gene_name": "Nucleoporin p54",
  "gene_symbol": "NUP54"
}